{
  "gene": "UniProtKB:Q9UPN3",
  "term_label": "cytoplasm",
  "gene_symbol": "MACF1",
  "gene_name": "Microtubule-actin cross-linking factor 1, isoforms 1_2_3_4_5",
  "term_id": "GO:0005737"
}